{
  "term_label": "transcription cis-regulatory region binding",
  "gene": "UniProtKB:Q8N393",
  "term_id": "GO:0000976",
  "gene_name": "Zinc finger protein 786",
  "gene_symbol": "ZNF786"
}